{
  "term_id": "GO:0007030",
  "term_label": "Golgi organization",
  "gene_symbol": "PI4K2A",
  "gene": "UniProtKB:Q9BTU6",
  "gene_name": "Phosphatidylinositol 4-kinase type 2-alpha"
}